{
  "term_label": "Unknown biological process",
  "gene": "UniProtKB:Q9HBJ0",
  "gene_name": "Placenta-specific protein 1",
  "term_id": "UNKNOWN:0002",
  "gene_symbol": "PLAC1"
}